{
  "gene_name": "Protein S100-A3",
  "gene": "UniProtKB:P33764",
  "term_label": "Unknown cellular component",
  "term_id": "UNKNOWN:0003",
  "gene_symbol": "S100A3"
}